{
  "gene_symbol": "STAT6",
  "term_id": "GO:0006952",
  "gene": "UniProtKB:P42226",
  "term_label": "defense response",
  "gene_name": "Signal transducer and activator of transcription 6"
}